blastoderm segmentation [GO:0007350] (biological process) Sources: ISBN:0879694238, http://fly.ebi.ac.uk/allied-data/lk/interactive-fly/aimain/1aahome.htm Relationships: is a type of embryonic pattern specification [GO:0009880]; is a type of GO:0035282 Definition: The hierarchical steps resulting in the progressive subdivision of the anterior/posterior axis of the embryo.